interleukin-18 receptor complex [GO:0045092] (cellular component) Relationships: is a type of plasma membrane signaling receptor complex [GO:0098802] References: PMID:12759435 Sources: GOC:mah Definition: A protein complex that binds interleukin-18; comprises an alpha and a beta subunit. Also known as: IL-18 receptor complex